{
  "term_label": "innate immune response",
  "gene_name": "E3 ubiquitin-protein ligase TRIM52",
  "term_id": "GO:0045087",
  "gene": "UniProtKB:Q96A61",
  "gene_symbol": "TRIM52"
}